{
  "gene_name": "Galanin receptor type 2",
  "gene_symbol": "GALR2",
  "term_id": "GO:0004966",
  "term_label": "galanin receptor activity",
  "gene": "UniProtKB:O43603"
}